{
  "gene_name": "Ubiquitin carboxyl-terminal hydrolase 6",
  "term_label": "cysteine-type deubiquitinase activity",
  "gene_symbol": "USP6",
  "term_id": "GO:0004843",
  "gene": "UniProtKB:P35125"
}